{
  "gene_name": "Ecotropic viral integration site 5 protein homolog",
  "gene_symbol": "EVI5",
  "term_label": "Unknown cellular component",
  "gene": "UniProtKB:O60447",
  "term_id": "UNKNOWN:0003"
}